{
  "term_label": "synapse",
  "gene_name": "Integrin beta-1",
  "gene_symbol": "ITGB1",
  "gene": "UniProtKB:P05556",
  "term_id": "GO:0045202"
}